high mobility group box 1 receptor activity [GO:0070380] (MF) Also known as: HMGB1 receptor activity References: PMID:18431461 Sources: GOC:add, GOC:signaling Relationships: is_a cytokine receptor activity [GO:0004896]; has part high mobility group box 1 binding [GO:0070379] Definition: Combining with high mobility group box 1 (HMBGB1) and transmitting the signal from one side of the membrane to the other to initiate a change in cell activity.